{
  "gene": "UniProtKB:B3SHH9",
  "gene_name": "Transmembrane protein 114",
  "gene_symbol": "TMEM114",
  "term_label": "Unknown biological process",
  "term_id": "UNKNOWN:0002"
}